{
  "term_label": "mitotic cell cycle",
  "term_id": "GO:0000278",
  "gene": "UniProtKB:P04350",
  "gene_symbol": "TUBB4A",
  "gene_name": "Tubulin beta-4A chain"
}